{
  "term_label": "RNA polymerase II cis-regulatory region sequence-specific DNA binding",
  "gene_symbol": "TBX2",
  "term_id": "GO:0000978",
  "gene": "UniProtKB:Q13207",
  "gene_name": "T-box transcription factor TBX2"
}